{
  "gene_symbol": "CFHR2",
  "gene_name": "Complement factor H-related protein 2",
  "term_label": "complement component C3b binding",
  "gene": "UniProtKB:P36980",
  "term_id": "GO:0001851"
}